{
  "gene_symbol": "CIC",
  "gene": "UniProtKB:Q96RK0",
  "gene_name": "Protein capicua homolog",
  "term_label": "RNA polymerase II transcription regulatory region sequence-specific DNA binding",
  "term_id": "GO:0000977"
}